{
  "gene": "UniProtKB:Q6ICB4",
  "gene_name": "Sesquipedalian-2",
  "term_id": "GO:0005802",
  "term_label": "trans-Golgi network",
  "gene_symbol": "PHETA2"
}